{
  "gene_symbol": "EHD3",
  "gene": "UniProtKB:Q9NZN3",
  "term_label": "endocytosis",
  "term_id": "GO:0006897",
  "gene_name": "EH domain-containing protein 3"
}